{
  "gene_name": "Tubulin-specific chaperone E",
  "gene": "UniProtKB:Q15813",
  "term_id": "GO:0007023",
  "term_label": "post-chaperonin tubulin folding pathway",
  "gene_symbol": "TBCE"
}